{
  "gene_symbol": "SLC24A5",
  "gene_name": "Sodium_potassium_calcium exchanger 5",
  "gene": "UniProtKB:Q71RS6",
  "term_id": "GO:0006874",
  "term_label": "intracellular calcium ion homeostasis"
}